long-chain fatty acyl-CoA hydrolase activity [GO:0052816] (molecular function) Definition: Catalysis of the reaction: a long-chain fatty acyl-CoA + H2O = a long-chain fatty acid + CoA + H+. A long-chain fatty acid has an aliphatic tail containing 13 to 22 carbons. Relationships: is a type of fatty acyl-CoA hydrolase activity [GO:0047617] Sources: RHEA:67680 Note: While there is not universal consensus on the lengths of short-, medium-, long- and very-long-chain fatty acids, the GO uses the definitions in ChEBI (see CHEBI:26666, CHEBI:59554, CHEBI:15904 and CHEBI:27283). Also known as: long-chain acyl coenzyme A hydrolase activity, long-chain acyl-thioester hydrolase activity, long-chain hydrolase activity, long-chain-acyl-CoA hydrolase activity